{
  "term_label": "nucleus",
  "gene": "UniProtKB:Q92988",
  "gene_symbol": "DLX4",
  "gene_name": "Homeobox protein DLX-4",
  "term_id": "GO:0005634"
}